{
  "gene": "UniProtKB:O95235",
  "gene_name": "Kinesin-like protein KIF20A",
  "term_id": "GO:0005874",
  "term_label": "microtubule",
  "gene_symbol": "KIF20A"
}